{
  "gene_name": "HLA class II histocompatibility antigen, DR beta 3 chain",
  "gene_symbol": "HLA-DRB3",
  "term_label": "positive regulation of T cell activation",
  "term_id": "GO:0050870",
  "gene": "UniProtKB:P79483"
}